{
  "gene": "UniProtKB:Q9Y5E9",
  "term_id": "GO:0005886",
  "term_label": "plasma membrane",
  "gene_name": "Protocadherin beta-14",
  "gene_symbol": "PCDHB14"
}